{
  "term_id": "GO:0004867",
  "gene": "UniProtKB:Q8TCV5",
  "gene_symbol": "WFDC5",
  "term_label": "serine-type endopeptidase inhibitor activity",
  "gene_name": "WAP four-disulfide core domain protein 5"
}